bacterial microcompartment [GO:0031469] (cellular component) Subtypes: GO:0031470, GO:0031471, propanediol degradation polyhedral organelle [GO:0031472] Also known as: BAC, BMC, MCP, polyhedral organelle References: PMID:10498708, PMID:11844753, PMID:12923081, PMID:34058518, PMID:34340100 Sources: GOC:js Definition: An organelle found in bacteria consisting of a proteinaceous coat containing metabolic enzymes whose purpose is the sequestration or concentration of metabolites and which has the appearance of a polygonal granule by electron microscopy. Relationships: is_a GO:0043232